{
  "term_label": "ubiquitin protein ligase activity",
  "gene_name": "RING-type domain-containing protein",
  "gene_symbol": "RNF228",
  "term_id": "GO:0061630",
  "gene": "UniProtKB:A0A7I2V3R4"
}